{
  "term_label": "Unknown cellular component",
  "gene": "UniProtKB:A0A0G2JKD1",
  "gene_symbol": "MUC21",
  "gene_name": "Mucin-21",
  "term_id": "UNKNOWN:0003"
}